growth factor complex [GO:0036454] (cellular component) Subtypes: insulin-like growth factor binding protein complex [GO:0016942], GO:1990150, platelet-derived growth factor complex [GO:1990265] Definition: A protein complex that has growth factor activity. Relationships: is a type of protein-containing complex [GO:0032991] Sources: GOC:bhm